{
  "term_label": "negative regulation of cell population proliferation",
  "gene": "UniProtKB:P42773",
  "gene_symbol": "CDKN2C",
  "gene_name": "Cyclin-dependent kinase 4 inhibitor C",
  "term_id": "GO:0008285"
}